{
  "gene": "UniProtKB:P12524",
  "gene_name": "Protein L-Myc",
  "term_label": "DNA-binding transcription factor activity, RNA polymerase II-specific",
  "term_id": "GO:0000981",
  "gene_symbol": "MYCL"
}